{
  "gene_name": "Formin-like protein 1",
  "gene_symbol": "FMNL1",
  "term_label": "cell migration",
  "term_id": "GO:0016477",
  "gene": "UniProtKB:O95466"
}